ABC-type azole transporter activity [GO:0140394] (molecular function) Also known as: azole ABC transporter activity, ATPase-coupled azole transmembrane transporter activity Subtypes: GO:0048502 Definition: Enables the transfer of azoles, heterocyclic compound found in many biologically important substances, from one side of a membrane to the other according to the reaction: ATP + H2O + azole(in) = ADP + phosphate + azole(out). Relationships: is_a GO:0140359; is a type of azole transmembrane transporter activity [GO:1901474] References: PMID:31501141 Sources: RHEA:33503